{
  "term_id": "GO:0008494",
  "term_label": "translation activator activity",
  "gene_name": "CBP80_20-dependent translation initiation factor",
  "gene_symbol": "CTIF",
  "gene": "UniProtKB:O43310"
}